{
  "gene_name": "Dystrophin",
  "gene": "UniProtKB:P11532",
  "gene_symbol": "DMD",
  "term_id": "GO:0099536",
  "term_label": "synaptic signaling"
}